{
  "gene_name": "Coiled-coil domain-containing protein 93",
  "gene_symbol": "CCDC93",
  "term_label": "Unknown molecular function",
  "gene": "UniProtKB:Q567U6",
  "term_id": "UNKNOWN:0001"
}